{
  "gene_symbol": "MPEG1",
  "gene_name": "Macrophage-expressed gene 1 protein",
  "gene": "UniProtKB:Q2M385",
  "term_label": "Unknown molecular function",
  "term_id": "UNKNOWN:0001"
}